glucosyl-N-acetylglucosamine glucosaminidase activity [GO:0052774] (molecular function) Relationships: is a type of GO:0015929 Definition: Catalysis of the reaction: glucosyl-N-acetylglucosamine + H2O = glucosamine + N-acetylglucosamine. References: PMID:15136574, PMID:16232910, PMID:16736587 Sources: GOC:mengo_curators